{
  "term_id": "GO:0008360",
  "gene_name": "Unconventional myosin-X",
  "term_label": "regulation of cell shape",
  "gene": "UniProtKB:Q9HD67",
  "gene_symbol": "MYO10"
}